positive regulation of cleistothecium development [GO:0070798] (biological process) Sources: GOC:mah Definition: Any process that activates or increases the frequency, rate or extent of cleistothecium development, a process that leads to the formation of a cleistothecium. The cleistothecium is a closed sexual fruiting body that contains ascospores in linear asci, characteristic of some filamentous Ascomycete fungi such as members of the genera Aspergillus and Emericella. Relationships: is a type of regulation of cleistothecium development [GO:0070796]; is a type of positive regulation of sporocarp development involved in sexual reproduction [GO:1902060]; positively regulates GO:0070791